{
  "gene_name": "Protein GDF5-AS1, mitochondrial",
  "term_label": "Unknown cellular component",
  "gene_symbol": "GDF5-AS1",
  "term_id": "UNKNOWN:0003",
  "gene": "UniProtKB:Q5U4N7"
}